{
  "term_label": "regulation of cell cycle",
  "gene_name": "Transcription factor JunD",
  "gene": "UniProtKB:P17535",
  "term_id": "GO:0051726",
  "gene_symbol": "JUND"
}